amacrine cell differentiation [GO:0035881] (biological process) Definition: The process in which a relatively unspecialized cell acquires specialized features of an amacrine cell, an interneuron generated in the inner nuclear layer (INL) of the vertebrate retina. Amacrine cells integrate, modulate, and interpose a temporal domain in the visual message presented to the retinal ganglion cells, with which they synapse in the inner plexiform layer. Amacrine cells lack large axons. Also known as: amacrine neuron differentiation Relationships: is a type of central nervous system neuron differentiation [GO:0021953]; is part of neural retina development [GO:0003407] Regulation: regulated by regulation of amacrine cell differentiation [GO:1902869]; negatively regulated by negative regulation of amacrine cell differentiation [GO:1902870]; positively regulated by positive regulation of amacrine cell differentiation [GO:1902871] Sources: CL:0000561, GOC:bf